galactose catabolic process via UDP-galactose, Leloir pathway [GO:0033499] (biological process) Also known as: Leloir Pathway, galactose breakdown via UDP-galactose, galactose catabolism via UDP-galactose, galactose degradation via UDP-galactose Sources: GOC:mah Definition: The chemical reactions and pathways resulting in the breakdown of galactose, via the intermediate UDP-galactose. Relationships: is a type of phosphate-containing compound metabolic process [GO:0006796]; is a type of GO:0019388; is a type of organophosphate catabolic process [GO:0046434]; is a type of carbohydrate derivative catabolic process [GO:1901136]